{
  "gene_symbol": "ALKBH5",
  "gene": "UniProtKB:Q6P6C2",
  "gene_name": "RNA demethylase ALKBH5",
  "term_label": "Unknown biological process",
  "term_id": "UNKNOWN:0002"
}